{
  "term_id": "GO:0030276",
  "gene_name": "MYCBP-associated protein",
  "gene": "UniProtKB:Q8TBZ2",
  "gene_symbol": "MYCBPAP",
  "term_label": "clathrin binding"
}